{
  "gene_name": "Kremen protein 1",
  "gene": "UniProtKB:Q96MU8",
  "term_label": "signal transduction",
  "gene_symbol": "KREMEN1",
  "term_id": "GO:0007165"
}